negative regulation of antifungal peptide secretion [GO:0002801] (biological process) Relationships: is a type of GO:0002789; is_a negative regulation of antimicrobial peptide secretion [GO:0002795]; is a type of GO:0002800; RO_0002212 antifungal peptide secretion [GO:0002782] Sources: GOC:add Definition: Any process that stops, prevents, or reduces the frequency, rate, or extent of antifungal peptide secretion. Also known as: down regulation of antifungal peptide secretion, down-regulation of antifungal peptide secretion, downregulation of antifungal peptide secretion, inhibition of antifungal peptide secretion